{
  "gene": "UniProtKB:P09693",
  "gene_name": "T-cell surface glycoprotein CD3 gamma chain",
  "term_id": "GO:0009897",
  "term_label": "external side of plasma membrane",
  "gene_symbol": "CD3G"
}